U12-type precatalytic spliceosome [GO:0071016] (cellular component) Also known as: minor precatalytic spliceosome, AT-AC precatalytic spliceosome, mammalian U12-type spliceosomal complex B, mammalian U12-type spliceosomal complex B1, yeast U12-type spliceosomal complex A2-1 Definition: A spliceosomal complex that is formed by the recruitment of the preassembled U4atac/U6atac.U5 tri-snRNP to the U12-type prespliceosome. Although all 5 snRNPs are present, the precatalytic spliceosome is catalytically inactive. The precatalytic spliceosome includes many proteins in addition to those found in the U11, U12 and U4atac/U6atac.U5 snRNPs. References: PMID:16201866 Sources: GOC:ab, GOC:krc, GOC:mah Relationships: is_a GO:0005689; is a type of precatalytic spliceosome [GO:0071011]; has part GO:0005692; has part U12 snRNP [GO:0005693]; has part U4atac/U6atac x U5 tri-snRNP complex [GO:0071009]